platelet alpha granule [GO:0031091] (cellular component) Also known as: platelet alpha-granule Definition: A secretory organelle found in blood platelets, which is unique in that it exhibits further compartmentalization and acquires its protein content via two distinct mechanisms: (1) biosynthesis predominantly at the megakaryocyte (MK) level (with some vestigial platelet synthesis) (e.g. platelet factor 4) and (2) endocytosis and pinocytosis at both the MK and circulating platelet levels (e.g. fibrinogen (Fg) and IgG). References: PMID:8467233 Relationships: is a type of secretory granule [GO:0030141]